{
  "term_id": "GO:0005886",
  "term_label": "plasma membrane",
  "gene": "UniProtKB:Q9Y345",
  "gene_name": "Sodium- and chloride-dependent glycine transporter 2",
  "gene_symbol": "SLC6A5"
}